{
  "term_label": "protein phosphatase binding",
  "gene_symbol": "CD22",
  "gene_name": "B-cell receptor CD22",
  "term_id": "GO:0019903",
  "gene": "UniProtKB:P20273"
}